histidine transport [GO:0015817] (BP) Relationships: is a type of basic amino acid transport [GO:0015802] Also known as: L-histidine transport Definition: The directed movement of histidine, 2-amino-3-(1H-imidazol-4-yl)propanoic acid, into, out of or within a cell, or between cells, by means of some agent such as a transporter or pore. Sources: GOC:ai